response to ziprasidone [GO:0097337] (biological process) Relationships: is a type of response to nitrogen compound [GO:1901698] Definition: Any process that results in a change in state or activity of a cell or an organism (in terms of movement, secretion, enzyme production, gene expression, etc.) as a result of a ziprasidone stimulus. Ziprasidone is a piperazine compound having 1,2-benzothiazol-3-yl- and 2-(6-chloro-1,3-dihydro-2-oxindol-5-yl)ethyl substituents attached to the nitrogen atoms. Sources: GOC:pr